{
  "gene_name": "Cyclin-C",
  "term_id": "GO:0016592",
  "term_label": "mediator complex",
  "gene_symbol": "CCNC",
  "gene": "UniProtKB:P24863"
}